immune response-inhibiting cell surface receptor signaling pathway [GO:0002767] (biological process) Relationships: is a type of immune response-inhibiting signal transduction [GO:0002765]; is a type of immune response-regulating cell surface receptor signaling pathway [GO:0002768] Definition: The series of molecular signals initiated by an extracellular ligand binding to a receptor on the surface of the target cell capable of inhibiting an immune response. References: PMID:15771571 Sources: GOC:add, ISBN:0781735149 Also known as: immune response-inhibiting cell surface receptor signalling pathway Subtypes: natural killer cell inhibitory signaling pathway [GO:0002769], T cell inhibitory signaling pathway [GO:0002770], inhibitory killer cell immunoglobulin-like receptor signaling pathway [GO:0002771], GO:0002772, B cell inhibitory signaling pathway [GO:0002773], GO:0002774